peripheral B cell anergy [GO:0002453] (biological process) Regulation: regulated by regulation of peripheral B cell anergy [GO:0002917]; negatively regulated by negative regulation of peripheral B cell anergy [GO:0002918]; positively regulated by positive regulation of peripheral B cell anergy [GO:0002919] Sources: GOC:jal, ISBN:0781735149 Definition: Any process contributing to anergy, a state of functional inactivation that occurs as part of tolerance induction, in peripheral B cells. Relationships: is a type of B cell anergy [GO:0002515]; is part of peripheral B cell tolerance induction [GO:0002451] Also known as: peripheral B lymphocyte anergy, peripheral B-cell anergy, peripheral B-lymphocyte anergy